{
  "term_id": "UNKNOWN:0003",
  "gene": "UniProtKB:Q8N888",
  "term_label": "Unknown cellular component",
  "gene_symbol": "BCORP1",
  "gene_name": "Putative BCoR-like protein 2"
}